positive regulation of urine volume by pressure natriuresis [GO:0035818] (biological process) Definition: An increase in the amount of urine excreted over a unit of time, as a result of pressure natriuresis. Sources: GOC:mtg_25march11, GOC:yaf Also known as: diuresis resulting from pressure natriuresis Relationships: is a type of pressure natriuresis [GO:0003095]; is a type of positive regulation of urine volume [GO:0035810]